{
  "term_id": "GO:0035529",
  "gene_name": "Nucleoside diphosphate-linked moiety X motif 17",
  "gene": "UniProtKB:P0C025",
  "term_label": "NADH pyrophosphatase activity",
  "gene_symbol": "NUDT17"
}